{
  "term_label": "spermidine biosynthetic process",
  "gene_symbol": "AMD1",
  "gene_name": "S-adenosylmethionine decarboxylase proenzyme",
  "term_id": "GO:0008295",
  "gene": "UniProtKB:P17707"
}